{
  "gene": "UniProtKB:Q99075",
  "gene_name": "Proheparin-binding EGF-like growth factor",
  "term_id": "GO:0008201",
  "gene_symbol": "HBEGF",
  "term_label": "heparin binding"
}